{
  "gene_symbol": "RNF24",
  "term_id": "UNKNOWN:0003",
  "gene": "UniProtKB:Q9Y225",
  "term_label": "Unknown cellular component",
  "gene_name": "RING finger protein 24"
}